{
  "gene_symbol": "PABPC4L",
  "gene": "UniProtKB:P0CB38",
  "term_id": "GO:0005829",
  "gene_name": "Polyadenylate-binding protein 4-like",
  "term_label": "cytosol"
}